{
  "term_label": "endosome",
  "gene": "UniProtKB:Q9NX40",
  "gene_name": "OCIA domain-containing protein 1",
  "term_id": "GO:0005768",
  "gene_symbol": "OCIAD1"
}